{
  "gene_name": "Putative uncharacterized protein FLJ40288",
  "gene_symbol": "A4D1N5",
  "gene": "UniProtKB:A4D1N5",
  "term_id": "UNKNOWN:0003",
  "term_label": "Unknown cellular component"
}